{
  "gene_symbol": "SPNS3",
  "term_id": "GO:0022857",
  "gene": "UniProtKB:Q6ZMD2",
  "term_label": "transmembrane transporter activity",
  "gene_name": "Protein spinster homolog 3"
}